response to sterol depletion [GO:0006991] (biological process) Subtypes: cellular response to sterol depletion [GO:0071501] Definition: Any process that results in a change in state or activity of a cell or an organism (in terms of movement, secretion, enzyme production, gene expression, etc.) as a result of a stimulus indicating deprivation of sterols. Sterols are a group of steroids characterized by the presence of one or more hydroxyl groups and a hydrocarbon side-chain in the molecule. Sources: GOC:bf, ISBN:0198506732 Also known as: sterol depletion response Relationships: is a type of GO:0006950